{
  "term_id": "GO:0043025",
  "gene": "UniProtKB:P43034",
  "gene_name": "Platelet-activating factor acetylhydrolase IB subunit beta",
  "term_label": "neuronal cell body",
  "gene_symbol": "PAFAH1B1"
}